{
  "gene_symbol": "LRRK2",
  "term_id": "GO:0035556",
  "term_label": "intracellular signal transduction",
  "gene_name": "Leucine-rich repeat serine_threonine-protein kinase 2",
  "gene": "UniProtKB:Q5S007"
}